{
  "gene": "UniProtKB:Q9NQ11",
  "term_id": "GO:0031902",
  "gene_symbol": "ATP13A2",
  "gene_name": "Polyamine-transporting ATPase 13A2",
  "term_label": "late endosome membrane"
}